{
  "gene_name": "Gliomedin",
  "term_label": "cell surface",
  "gene_symbol": "GLDN",
  "term_id": "GO:0009986",
  "gene": "UniProtKB:Q6ZMI3"
}